{
  "gene": "UniProtKB:Q9P0W0",
  "gene_symbol": "IFNK",
  "term_label": "cytokine activity",
  "term_id": "GO:0005125",
  "gene_name": "Interferon kappa"
}